protein localization to plasma membrane [GO:0072659] (biological process) Also known as: protein localisation in plasma membrane, protein localization in plasma membrane, protein targeting to plasma membrane, protein-plasma membrane targeting Definition: A process in which a protein is transported to, or maintained in, a specific location in the plasma membrane. Relationships: is a type of protein localization to membrane [GO:0072657]; is a type of protein localization to cell periphery [GO:1990778] Subtypes: protein localization to T-tubule [GO:0036371], Golgi to plasma membrane protein transport [GO:0043001], endosome to plasma membrane protein transport [GO:0099638], protein transport from ciliary membrane to plasma membrane [GO:1903445] Regulation: RO_0002211 by regulation of protein localization to plasma membrane [GO:1903076]; negatively regulated by negative regulation of protein localization to plasma membrane [GO:1903077]; positively regulated by GO:1903078 Sources: GOC:mah